{
  "gene_symbol": "NXPE1",
  "term_id": "UNKNOWN:0001",
  "gene": "UniProtKB:Q8N323",
  "gene_name": "NXPE family member 1",
  "term_label": "Unknown molecular function"
}